positive regulation of establishment of RNA localization to telomere [GO:1904912] (biological process) Definition: Any process that activates or increases the frequency, rate or extent of establishment of RNA localization to telomere. References: PMID:26586433 Sources: GOC:BHF, GOC:BHF_telomere, GOC:TermGenie, GOC:rph, GO_REF:0000058 Also known as: positive regulation of establishment of RNA localisation to telomere, up regulation of establishment of RNA localisation to telomere, up regulation of establishment of RNA localization to telomere, up-regulation of establishment of RNA localisation to telomere, up-regulation of establishment of RNA localization to telomere, upregulation of establishment of RNA localisation to telomere, upregulation of establishment of RNA localization to telomere, activation of establishment of RNA localisation to telomere, activation of establishment of RNA localization to telomere Relationships: is a type of positive regulation of biological process [GO:0048518]; is a type of regulation of establishment of RNA localization to telomere [GO:1904910]; positively regulates GO:0097694